{
  "gene": "UniProtKB:P10767",
  "gene_symbol": "FGF6",
  "term_id": "GO:0008083",
  "term_label": "growth factor activity",
  "gene_name": "Fibroblast growth factor 6"
}